{
  "term_id": "GO:0005886",
  "gene_name": "C5a anaphylatoxin chemotactic receptor 1",
  "gene_symbol": "C5AR1",
  "term_label": "plasma membrane",
  "gene": "UniProtKB:P21730"
}